{
  "gene": "UniProtKB:Q9NXL6",
  "term_id": "GO:0050658",
  "gene_symbol": "SIDT1",
  "gene_name": "SID1 transmembrane family member 1",
  "term_label": "RNA transport"
}